{
  "term_label": "positive regulation of mitochondrial calcium ion concentration",
  "gene_symbol": "MCUR1",
  "gene_name": "Mitochondrial calcium uniporter regulator 1",
  "term_id": "GO:0051561",
  "gene": "UniProtKB:Q96AQ8"
}